{
  "term_id": "GO:0070888",
  "gene": "UniProtKB:Q13516",
  "gene_name": "Oligodendrocyte transcription factor 2",
  "term_label": "E-box binding",
  "gene_symbol": "OLIG2"
}